diuretic hormone receptor activity [GO:0008036] (molecular function) Definition: Combining with a diuretic hormone and transmitting the signal to initiate a change in cell activity. Sources: GOC:ai, GOC:signaling Relationships: is a type of GO:0038023; is part of hormone-mediated signaling pathway [GO:0009755]